platelet-activating factor acetyltransferase activity [GO:0047179] (molecular function) Definition: Catalysis of the reaction: 1-radyl-2-acyl-sn-glycero-3-phospholipid + 1-alkyl-2-acetyl-sn-glycero-3-phosphocholine = 1-alkyl-2-lyso-sn-glycero-3-phosphocholine + 1-radyl-2-acetyl-sn-glycero-3-phospholipid. Sources: EC:2.3.1.149, MetaCyc:2.3.1.149-RXN Also known as: PAF acetyltransferase activity, 1-alkyl-2-acyl-sn-glycero-3-phosphocholine:1-organyl-2-lyso-sn-glycero-3-phospholipid acetyltransferase activity Relationships: is a type of acetyltransferase activity [GO:0016407]